{
  "term_label": "Unknown molecular function",
  "gene_symbol": "PYY2",
  "gene_name": "Putative peptide YY-2",
  "term_id": "UNKNOWN:0001",
  "gene": "UniProtKB:Q9NRI6"
}